{
  "term_label": "Unknown molecular function",
  "term_id": "UNKNOWN:0001",
  "gene": "UniProtKB:O95183",
  "gene_name": "Vesicle-associated membrane protein 5",
  "gene_symbol": "VAMP5"
}